{
  "gene": "UniProtKB:Q9UN81",
  "gene_symbol": "L1RE1",
  "gene_name": "LINE-1 retrotransposable element ORF1 protein",
  "term_label": "single-stranded RNA binding",
  "term_id": "GO:0003727"
}